ganglion development [GO:0061548] (biological process) Also known as: gangliogenesis, ganglia development Relationships: is_a tissue development [GO:0009888]; is part of GO:0007399 Definition: The process whose specific outcome is the progression of a ganglion over time, from its formation to the mature structure. Sources: GOC:dph Subtypes: GO:0061549, cranial ganglion development [GO:0061550], dorsal root ganglion development [GO:1990791]